{
  "term_label": "membrane",
  "gene": "UniProtKB:Q96SL1",
  "term_id": "GO:0016020",
  "gene_symbol": "SLC49A4",
  "gene_name": "Solute carrier family 49 member 4"
}